{
  "term_id": "GO:0019814",
  "gene_name": "Immunoglobulin lambda variable 3-16",
  "term_label": "immunoglobulin complex",
  "gene_symbol": "IGLV3-16",
  "gene": "UniProtKB:A0A075B6K0"
}